{
  "gene": "UniProtKB:Q8IWR0",
  "gene_symbol": "ZC3H7A",
  "gene_name": "Zinc finger CCCH domain-containing protein 7A",
  "term_id": "GO:0035198",
  "term_label": "miRNA binding"
}